movement of group I intron [GO:0006316] (BP) Definition: Lateral transfer of a group I intron to a homologous allele that lacks the intron, mediated by a site-specific endonuclease encoded within the mobile intron; group I introns are self-splicing introns that use guanosine as a cofactor in the splicing reaction. References: PMID:10487208 Sources: GOC:mcc, ISBN:0716743663 Relationships: is a type of intron homing [GO:0006314]